{
  "gene": "UniProtKB:Q9HAA7",
  "term_label": "Unknown cellular component",
  "gene_symbol": "Q9HAA7",
  "gene_name": "Putative uncharacterized protein FLJ11871",
  "term_id": "UNKNOWN:0003"
}